MAP kinase activity [GO:0004707] (molecular function) Also known as: ERK1, mitogen activated kinase activity, MAP kinase 1 activity, MAP kinase 2 activity, MBP kinase I activity, MBP kinase II activity, SAP kinase activity, SAPK, extracellular signal-regulated kinase activity, myelin basic protein kinase activity, stress-activated kinase activity, stress-activated protein kinase activity, ATP:protein phosphotransferase (MAPKK-activated) activity, ERK, ERK2, MAPK, mitogen-activated protein kinase activity Regulation: regulated by GO:0043405; positively regulated by positive regulation of MAP kinase activity [GO:0043406]; negatively regulated by negative regulation of MAP kinase activity [GO:0043407] Subtypes: GO:0004705 Sources: GOC:ma, ISBN:0198547684 Definition: Catalysis of the reaction: protein + ATP = protein phosphate + ADP. This reaction is the phosphorylation of proteins. Mitogen-activated protein kinase; a family of protein kinases that perform a crucial step in relaying signals from the plasma membrane to the nucleus. They are activated by a wide range of proliferation- or differentiation-inducing signals; activation is strong with agonists such as polypeptide growth factors and tumor-promoting phorbol esters, but weak (in most cell backgrounds) by stress stimuli. Relationships: is a type of protein serine/threonine kinase activity [GO:0004674]; is part of MAPK cascade [GO:0000165]